{
  "gene_symbol": "GANAB",
  "gene": "UniProtKB:Q14697",
  "term_id": "GO:0006491",
  "gene_name": "Neutral alpha-glucosidase AB",
  "term_label": "N-glycan processing"
}